{
  "gene_symbol": "UBQLN1",
  "gene": "UniProtKB:Q9UMX0",
  "term_id": "GO:0036503",
  "term_label": "ERAD pathway",
  "gene_name": "Ubiquilin-1"
}